{
  "gene_name": "Keratin-associated protein 10-9",
  "term_id": "UNKNOWN:0002",
  "term_label": "Unknown biological process",
  "gene": "UniProtKB:P60411",
  "gene_symbol": "KRTAP10-9"
}